cystathionine gamma-synthase activity [GO:0003962] (molecular function) Sources: RHEA:20397 Definition: Catalysis of the reaction: L-cysteine + O-succinyl-L-homoserine = H+ + L,L-cystathionine + succinate. Relationships: is_a transferase activity, transferring alkyl or aryl (other than methyl) groups [GO:0016765] Also known as: homoserine O-transsuccinylase activity, homoserine transsuccinylase activity, CTT gamma synthase activity, O-succinyl-L-homoserine (thiol)-lyase activity, O-succinyl-L-homoserine succinate-lyase activity, cystathionine g-synthase activity, cystathionine gamma synthase activity, cystathionine gamma-synthase activity (acts on O-phosphohomoserine), O-succinyl-L-homoserine succinate-lyase (adding cysteine) activity, O-succinylhomoserine (thiol)-lyase activity, O-succinylhomoserine synthase activity, O-succinylhomoserine synthetase activity, O4-succinyl-L-homoserine:L-cysteine S-(3-amino-3-carboxypropyl)transferase activity, cystathionine synthase activity, cystathionine synthetase activity